{
  "gene": "UniProtKB:Q9Y485",
  "term_id": "GO:0043291",
  "gene_name": "DmX-like protein 1",
  "gene_symbol": "DMXL1",
  "term_label": "RAVE complex"
}